RNA polymerase II transcription initiation surveillance [GO:0160240] (biological process) Relationships: is a type of GO:0071027; is part of transcription initiation at RNA polymerase II promoter [GO:0006367] References: PMID:33385327, PMID:34762484 Definition: A process that promotes premature RNA polymerase II transcription termination of transcripts that are unfavorably configured for transcriptional elongation by releasing RNA polymerase II from bound DNA or promoting RNA polymerase II degradation.